{
  "term_label": "Unknown biological process",
  "gene_symbol": "ZDHHC13",
  "gene": "UniProtKB:Q8IUH4",
  "term_id": "UNKNOWN:0002",
  "gene_name": "Palmitoyltransferase ZDHHC13"
}